{
  "gene": "UniProtKB:P18564",
  "gene_symbol": "ITGB6",
  "gene_name": "Integrin beta-6",
  "term_id": "GO:0007160",
  "term_label": "cell-matrix adhesion"
}